ESCRT IV complex [GO:1990621] (cellular component) Also known as: ESCRT-IV, VPS4A-VPS4B, VPS4A/B complex, Vps4-Vta1 complex, Vps4 complex, Vta1-Vps4 complex, vacuolar protein sorting-associated complex References: PMID:20653365, PMID:20696398, PMID:21925211, PMID:24456136, PMID:25164817, PMID:26775243 Sources: GOC:bhm, GOC:ha Relationships: is a type of ESCRT complex [GO:0036452]; is a type of membrane protein complex [GO:0098796]; is_a ATPase complex [GO:1904949]; BFO_0000050 GO:0010008 Definition: An ESCRT complex that has AAA-ATPase activity and is involved in ESCRT-mediated intralumenal vesicle formation and the final stages of cytokinesis. The complex catalyzes disassembly of the ESCRT III filament around the neck of the budding vesicle in an ATP-driven reaction, resulting in membrane scission and recycling of the ESCRT III components back to the cytosol. In yeast, it is formed by the AAA ATPase Vps4 and its cofactor Vta1.